{
  "gene": "UniProtKB:A0A0J9YXA8",
  "gene_symbol": "TRBJ1-1",
  "term_id": "UNKNOWN:0001",
  "term_label": "Unknown molecular function",
  "gene_name": "T cell receptor beta joining 1-1"
}